{
  "gene_symbol": "CHRNA9",
  "term_id": "GO:0045202",
  "term_label": "synapse",
  "gene": "UniProtKB:Q9UGM1",
  "gene_name": "Neuronal acetylcholine receptor subunit alpha-9"
}